positive regulation of stress fiber assembly [GO:0051496] (biological process) Definition: Any process that activates or increases the frequency, rate or extent of the assembly of a stress fiber, a bundle of microfilaments and other proteins found in fibroblasts. Also known as: up-regulation of stress fiber formation, activation of stress fiber formation, stimulation of stress fiber formation, positive regulation of stress fibre biosynthesis, positive regulation of stress fibre formation, up regulation of stress fiber formation, upregulation of stress fiber formation Relationships: is a type of positive regulation of actin filament bundle assembly [GO:0032233]; is a type of GO:0051492; positively regulates stress fiber assembly [GO:0043149] Sources: GOC:ai